{
  "term_id": "GO:1903119",
  "gene_name": "Filamin A-interacting protein 1-like",
  "term_label": "protein localization to actin cytoskeleton",
  "gene": "UniProtKB:Q4L180",
  "gene_symbol": "FILIP1L"
}